{
  "gene_symbol": "DPYSL3",
  "gene": "UniProtKB:Q14195",
  "term_id": "GO:0016812",
  "term_label": "hydrolase activity, acting on carbon-nitrogen (but not peptide) bonds, in cyclic amides",
  "gene_name": "Dihydropyrimidinase-related protein 3"
}